positive regulation of Schwann cell proliferation involved in axon regeneration [GO:1905046] (biological process) References: PMID:22393241 Sources: GOC:BHF, GOC:BHF_miRNA, GOC:TermGenie, GOC:rph, GO_REF:0000058 Also known as: up regulation of Schwann cell proliferation involved in axon regeneration, up-regulation of Schwann cell proliferation involved in axon regeneration, upregulation of Schwann cell proliferation involved in axon regeneration, activation of Schwann cell proliferation involved in axon regeneration Relationships: is a type of positive regulation of Schwann cell proliferation [GO:0010625]; is_a regulation of Schwann cell proliferation involved in axon regeneration [GO:1905044]; RO_0002213 Schwann cell proliferation involved in axon regeneration [GO:0014011] Definition: Any process that activates or increases the frequency, rate or extent of Schwann cell proliferation involved in axon regeneration.